{
  "gene": "UniProtKB:P41595",
  "term_id": "GO:0030425",
  "gene_name": "5-hydroxytryptamine receptor 2B",
  "gene_symbol": "HTR2B",
  "term_label": "dendrite"
}